{
  "term_label": "transmembrane signaling receptor activity",
  "gene_symbol": "MRC2",
  "gene_name": "C-type mannose receptor 2",
  "gene": "UniProtKB:Q9UBG0",
  "term_id": "GO:0004888"
}